{
  "gene_symbol": "OR51B6",
  "term_id": "UNKNOWN:0002",
  "gene": "UniProtKB:Q9H340",
  "term_label": "Unknown biological process",
  "gene_name": "Olfactory receptor 51B6"
}